{
  "gene_name": "Palmitoyltransferase ZDHHC12",
  "term_label": "protein targeting to membrane",
  "gene_symbol": "ZDHHC12",
  "term_id": "GO:0006612",
  "gene": "UniProtKB:Q96GR4"
}